{
  "gene_symbol": "GEM",
  "term_label": "GTP binding",
  "term_id": "GO:0005525",
  "gene": "UniProtKB:P55040",
  "gene_name": "GTP-binding protein GEM"
}